{
  "term_id": "GO:0008017",
  "gene_name": "Kinesin-like protein KIF13A",
  "gene_symbol": "KIF13A",
  "term_label": "microtubule binding",
  "gene": "UniProtKB:Q9H1H9"
}